{
  "gene": "UniProtKB:P54646",
  "term_id": "GO:0005737",
  "gene_name": "5'-AMP-activated protein kinase catalytic subunit alpha-2",
  "term_label": "cytoplasm",
  "gene_symbol": "PRKAA2"
}